{
  "gene_name": "Interleukin-10 receptor subunit alpha",
  "gene_symbol": "IL10RA",
  "term_id": "GO:0019221",
  "gene": "UniProtKB:Q13651",
  "term_label": "cytokine-mediated signaling pathway"
}